{
  "term_id": "UNKNOWN:0002",
  "term_label": "Unknown biological process",
  "gene": "UniProtKB:Q6MZN7",
  "gene_symbol": "HCP5",
  "gene_name": "HLA class I histocompatibility antigen protein P5"
}